{
  "gene_symbol": "OPN1SW",
  "term_label": "G protein-coupled receptor signaling pathway",
  "gene_name": "Short-wave-sensitive opsin 1",
  "term_id": "GO:0007186",
  "gene": "UniProtKB:P03999"
}